{
  "term_id": "UNKNOWN:0002",
  "gene_name": "Dendritic cell nuclear protein 1",
  "gene": "UniProtKB:Q8TF63",
  "gene_symbol": "DCANP1",
  "term_label": "Unknown biological process"
}